{
  "gene": "UniProtKB:A6NCS4",
  "gene_symbol": "NKX2-6",
  "term_label": "DNA-binding transcription factor activity, RNA polymerase II-specific",
  "term_id": "GO:0000981",
  "gene_name": "Homeobox protein Nkx-2.6"
}